{
  "gene": "UniProtKB:Q6ZTA4",
  "gene_name": "Tripartite motif-containing protein 67",
  "gene_symbol": "TRIM67",
  "term_label": "Unknown molecular function",
  "term_id": "UNKNOWN:0001"
}